oral/aboral axis specification [GO:0060834] (biological process) Definition: The establishment, maintenance and elaboration of a line that delineates the mouth and the anus of an embryo. Sources: GOC:dph, GOC:sdb_2009, GOC:tb Also known as: oral/aboral axis determination Relationships: is a type of embryonic axis specification [GO:0000578]